{
  "term_id": "GO:0000387",
  "gene_name": "Small nuclear ribonucleoprotein Sm D3",
  "gene_symbol": "SNRPD3",
  "gene": "UniProtKB:P62318",
  "term_label": "spliceosomal snRNP assembly"
}